{
  "term_id": "GO:0035556",
  "gene_symbol": "PKN3",
  "gene": "UniProtKB:Q6P5Z2",
  "gene_name": "Serine_threonine-protein kinase N3",
  "term_label": "intracellular signal transduction"
}